{
  "term_label": "nucleus",
  "gene_symbol": "PPM1F",
  "gene": "UniProtKB:P49593",
  "gene_name": "Protein phosphatase 1F",
  "term_id": "GO:0005634"
}